{
  "gene_symbol": "SUB1",
  "term_id": "GO:0005634",
  "term_label": "nucleus",
  "gene": "UniProtKB:P53999",
  "gene_name": "Activated RNA polymerase II transcriptional coactivator p15"
}